{
  "term_id": "GO:0009134",
  "gene": "UniProtKB:P49961",
  "term_label": "nucleoside diphosphate catabolic process",
  "gene_symbol": "ENTPD1",
  "gene_name": "Ectonucleoside triphosphate diphosphohydrolase 1"
}